{
  "term_label": "ceramide 1-phosphate binding",
  "gene_symbol": "GLTPD2",
  "term_id": "GO:1902387",
  "gene_name": "Glycolipid transfer protein domain-containing protein 2",
  "gene": "UniProtKB:A6NH11"
}